{
  "gene_symbol": "PGGHG",
  "term_id": "GO:0005975",
  "term_label": "carbohydrate metabolic process",
  "gene": "UniProtKB:Q32M88",
  "gene_name": "Protein-glucosylgalactosylhydroxylysine glucosidase"
}